dinucleotide repeat insertion binding [GO:0032181] (molecular function) Definition: Binding to a double-stranded DNA region containing a dinucleotide repeat insertion or a deletion resulting in unpaired dinucleotide repeats. Sources: GOC:mah, GOC:vk Relationships: is a type of GO:0032139